Actinobacterium-type cell wall biogenesis [GO:0071766] (biological process) Definition: A cellular process that results in the biosynthesis of constituent macromolecules, assembly, and arrangement of constituent parts of a cell wall of the type found in Actinobacteria. The cell wall is the rigid or semi-rigid envelope lying outside the cell membrane. Actinobacterial cell walls contain characteristic mycolic acids, of which some are covalently linked to the cell wall peptidoglycan and others accumulate at the cell surface. Relationships: is a type of peptidoglycan-based cell wall biogenesis [GO:0009273] References: PMID:15653820, PMID:3149973 Sources: GOC:mah